{
  "gene": "UniProtKB:Q6ZMB5",
  "term_id": "GO:0031901",
  "term_label": "early endosome membrane",
  "gene_symbol": "TMEM184A",
  "gene_name": "Transmembrane protein 184A"
}